{
  "term_id": "GO:0000015",
  "term_label": "phosphopyruvate hydratase complex",
  "gene_symbol": "ENO2",
  "gene": "UniProtKB:P09104",
  "gene_name": "Gamma-enolase"
}